NAD-dependent protein lysine delactylase activity [GO:0141208] (molecular function) Relationships: is a type of NAD-dependent protein lysine deacetylase activity [GO:0034979] References: PMID:38512451 Sources: RHEA:80287 Also known as: protein lysine delactylase activity Definition: Catalysis of the reaction: H2O + N6-lactoyl-L-lysyl-[protein] + NAD = L-lysyl-[protein] + nicotinamide +2''-O-lactoyl-ADP-D-ribose, transfering a lactoyl group attached to a lysine residue in a protein to NAD.